{
  "gene_symbol": "RGS6",
  "gene": "UniProtKB:P49758",
  "term_id": "GO:0005096",
  "term_label": "GTPase activator activity",
  "gene_name": "Regulator of G-protein signaling 6"
}